{
  "gene": "UniProtKB:Q96CN9",
  "term_label": "Golgi apparatus",
  "term_id": "GO:0005794",
  "gene_symbol": "GCC1",
  "gene_name": "GRIP and coiled-coil domain-containing protein 1"
}